{
  "term_label": "cellular response to lipopolysaccharide",
  "gene": "UniProtKB:Q15025",
  "gene_symbol": "TNIP1",
  "gene_name": "TNFAIP3-interacting protein 1",
  "term_id": "GO:0071222"
}